{
  "term_id": "UNKNOWN:0001",
  "gene_name": "Putative uncharacterized protein BAALC-AS2",
  "gene_symbol": "BAALC-AS2",
  "gene": "UniProtKB:P0C853",
  "term_label": "Unknown molecular function"
}